{
  "gene": "UniProtKB:Q13133",
  "term_label": "positive regulation of transcription by RNA polymerase II",
  "gene_name": "Oxysterols receptor LXR-alpha",
  "term_id": "GO:0045944",
  "gene_symbol": "NR1H3"
}